polysialic-acid O-acetyltransferase activity [GO:0050208] (molecular function) Sources: EC:2.3.1.136, MetaCyc:POLYSIALIC-ACID-O-ACETYLTRANSFERASE-RXN Relationships: is a type of O-acetyltransferase activity [GO:0016413] Also known as: acetyl-CoA:polysialic-acid O-acetyltransferase activity Definition: Catalysis of the reaction: acetyl-CoA + an alpha-2,8-linked polymer of sialic acid = CoA + polysialic acid acetylated at O-7 or O-9.